{
  "gene_symbol": "CST11",
  "term_label": "nucleus",
  "term_id": "GO:0005634",
  "gene": "UniProtKB:Q9H112",
  "gene_name": "Cystatin-11"
}